negative regulation of MyD88-dependent toll-like receptor signaling pathway [GO:0034125] (biological process) Relationships: is a type of negative regulation of toll-like receptor signaling pathway [GO:0034122]; is a type of regulation of MyD88-dependent toll-like receptor signaling pathway [GO:0034124]; negatively regulates MyD88-dependent toll-like receptor signaling pathway [GO:0002755] Definition: Any process that stops, prevents, or reduces the frequency, rate, or extent of MyD88-dependent toll-like receptor signaling pathway. References: PMID:16551253, PMID:17328678 Sources: GOC:add Also known as: negative regulation of MyD88-dependent TLR signaling pathway, negative regulation of MyD88-dependent toll-like receptor signalling pathway